{
  "gene_name": "Protein myomixer",
  "gene_symbol": "MYMX",
  "gene": "UniProtKB:A0A1B0GTQ4",
  "term_label": "Unknown molecular function",
  "term_id": "UNKNOWN:0001"
}